{
  "gene_symbol": "GUCY2C",
  "term_id": "GO:0006182",
  "gene": "UniProtKB:P25092",
  "gene_name": "Guanylyl cyclase C",
  "term_label": "cGMP biosynthetic process"
}